{
  "gene": "UniProtKB:P08581",
  "gene_symbol": "MET",
  "term_label": "hepatocyte growth factor receptor activity",
  "term_id": "GO:0005008",
  "gene_name": "Hepatocyte growth factor receptor"
}